{
  "term_label": "epithelial cell differentiation",
  "gene_name": "Keratin, type I cytoskeletal 9",
  "gene_symbol": "KRT9",
  "gene": "UniProtKB:P35527",
  "term_id": "GO:0030855"
}